regulation of aflatoxin biosynthetic process [GO:1900177] (BP) Also known as: regulation of aflatoxin anabolism, regulation of aflatoxin biosynthesis, regulation of aflatoxin formation, regulation of aflatoxin synthesis Definition: Any process that modulates the frequency, rate or extent of aflatoxin biosynthetic process. Sources: GOC:di Relationships: is a type of GO:0062012; is a type of regulation of secondary metabolite biosynthetic process [GO:1900376]; regulates aflatoxin biosynthetic process [GO:0045122] Subtypes: negative regulation of aflatoxin biosynthetic process [GO:1900178], positive regulation of aflatoxin biosynthetic process [GO:1900179]